{
  "gene_symbol": "DBP",
  "term_id": "GO:0005634",
  "gene_name": "D site-binding protein",
  "term_label": "nucleus",
  "gene": "UniProtKB:Q10586"
}